{
  "term_label": "Unknown biological process",
  "gene": "UniProtKB:P14854",
  "gene_name": "Cytochrome c oxidase subunit 6B1",
  "term_id": "UNKNOWN:0002",
  "gene_symbol": "COX6B1"
}